{
  "gene_symbol": "GLOD4",
  "term_id": "UNKNOWN:0002",
  "gene": "UniProtKB:Q9HC38",
  "term_label": "Unknown biological process",
  "gene_name": "Glyoxalase domain-containing protein 4"
}